{
  "term_label": "inflammatory response",
  "gene_symbol": "TLR2",
  "gene_name": "Toll-like receptor 2",
  "gene": "UniProtKB:O60603",
  "term_id": "GO:0006954"
}